{
  "term_label": "extracellular space",
  "gene_symbol": "INSL3",
  "term_id": "GO:0005615",
  "gene": "UniProtKB:P51460",
  "gene_name": "Insulin-like 3"
}